{
  "term_id": "GO:0030141",
  "gene_symbol": "STXBP2",
  "term_label": "secretory granule",
  "gene": "UniProtKB:Q15833",
  "gene_name": "Syntaxin-binding protein 2"
}